{
  "term_id": "GO:0008139",
  "gene_symbol": "IPO5",
  "gene": "UniProtKB:O00410",
  "term_label": "nuclear localization sequence binding",
  "gene_name": "Importin-5"
}